{
  "gene": "UniProtKB:P23771",
  "gene_symbol": "GATA3",
  "term_id": "GO:0045165",
  "term_label": "cell fate commitment",
  "gene_name": "Trans-acting T-cell-specific transcription factor GATA-3"
}